{
  "gene_symbol": "BCL2L12",
  "term_label": "negative regulation of intrinsic apoptotic signaling pathway in response to DNA damage by p53 class mediator",
  "gene": "UniProtKB:Q9HB09",
  "term_id": "GO:1902166",
  "gene_name": "Bcl-2-like protein 12"
}